{
  "gene_name": "1-phosphatidylinositol 4,5-bisphosphate phosphodiesterase beta-2",
  "gene_symbol": "PLCB2",
  "gene": "UniProtKB:Q00722",
  "term_label": "phosphatidylinositol metabolic process",
  "term_id": "GO:0046488"
}